{
  "gene_symbol": "AGTR1",
  "term_id": "GO:0006954",
  "gene": "UniProtKB:P30556",
  "term_label": "inflammatory response",
  "gene_name": "Type-1 angiotensin II receptor"
}